{
  "term_id": "GO:0010820",
  "gene": "UniProtKB:Q9UEW8",
  "gene_symbol": "STK39",
  "gene_name": "STE20_SPS1-related proline-alanine-rich protein kinase",
  "term_label": "positive regulation of T cell chemotaxis"
}